{
  "gene_name": "Histone chaperone ASF1B",
  "gene": "UniProtKB:Q9NVP2",
  "term_label": "DNA replication-dependent chromatin assembly",
  "gene_symbol": "ASF1B",
  "term_id": "GO:0006335"
}